sweet taste receptor complex [GO:1903767] (cellular component) Relationships: is a type of taste receptor complex [GO:1903768] References: PMID:16720576 Sources: GOC:BHF, GOC:TermGenie, GOC:rl, GO_REF:0000088 Definition: A protein complex which is capable of sweet taste receptor activity.